{
  "term_id": "GO:0035023",
  "gene_symbol": "ARHGEF2",
  "term_label": "regulation of Rho protein signal transduction",
  "gene_name": "Rho guanine nucleotide exchange factor 2",
  "gene": "UniProtKB:Q92974"
}